{
  "gene": "UniProtKB:Q9Y6P5",
  "gene_symbol": "SESN1",
  "term_id": "GO:1904262",
  "term_label": "negative regulation of TORC1 signaling",
  "gene_name": "Sestrin-1"
}